{
  "term_id": "GO:0000981",
  "gene_name": "Transcription factor Dp-1",
  "gene_symbol": "TFDP1",
  "term_label": "DNA-binding transcription factor activity, RNA polymerase II-specific",
  "gene": "UniProtKB:Q14186"
}